substantia propria of cornea development [GO:1903701] (biological process) Also known as: corneal stroma development, stroma of cornea development, substantia propria development References: PMID:12556382 Sources: GOC:TermGenie, GO_REF:0000094 Definition: The process whose specific outcome is the progression of a substantia propria of cornea over time, from its formation to the mature structure. Relationships: is a type of anatomical structure development [GO:0048856]